{
  "gene_name": "Leucine-rich repeat-containing protein 3",
  "term_id": "UNKNOWN:0001",
  "gene_symbol": "LRRC3",
  "term_label": "Unknown molecular function",
  "gene": "UniProtKB:Q9BY71"
}